metanephric mesenchymal cell differentiation [GO:0072162] (biological process) Sources: GOC:mtg_kidney_jan10 Relationships: is a type of mesenchymal cell differentiation involved in kidney development [GO:0072161]; is a type of cell differentiation involved in metanephros development [GO:0072202]; is part of metanephric mesenchyme development [GO:0072075] Definition: The process in which relatively unspecialized cells acquire specialized structural and/or functional features that characterize the mesenchymal cells of the metanephros as it progresses from its formation to the mature state.